{
  "term_id": "GO:0005509",
  "gene_symbol": "CALU",
  "term_label": "calcium ion binding",
  "gene": "UniProtKB:O43852",
  "gene_name": "Calumenin"
}